{
  "gene": "UniProtKB:Q96AX1",
  "term_id": "GO:0016192",
  "gene_symbol": "VPS33A",
  "gene_name": "Vacuolar protein sorting-associated protein 33A",
  "term_label": "vesicle-mediated transport"
}